{
  "gene_name": "Semaphorin-3B",
  "term_label": "neural crest cell migration",
  "term_id": "GO:0001755",
  "gene": "UniProtKB:Q13214",
  "gene_symbol": "SEMA3B"
}